ammonia assimilation cycle [GO:0019676] (biological process) Regulation: regulated by GO:2001248; negatively regulated by negative regulation of ammonia assimilation cycle [GO:2001249]; positively regulated by positive regulation of ammonia assimilation cycle [GO:2001250] Also known as: glutamate metabolic process via glutamine and ammonia, glutamate metabolism via glutamine and ammonia Relationships: is a type of glutamate metabolic process [GO:0006536]; is a type of GO:0006541; is a type of GO:0019740 Definition: The pathway by which ammonia is processed and incorporated into a cell. In an energy-rich (glucose-containing), nitrogen-poor environment, glutamine synthetase and glutamate synthase form an ammonia assimilatory cycle, in which ammonia is incorporated into L-glutamate to form L-glutamine, which then combines with alpha-ketoglutarate to regenerate L-glutamate. This ATP-dependent cycle is essential for nitrogen-limited growth and for steady-state growth with some sources of nitrogen. Sources: MetaCyc:AMMASSIM-PWY